{
  "term_id": "GO:1905475",
  "gene": "UniProtKB:Q8N158",
  "term_label": "regulation of protein localization to membrane",
  "gene_symbol": "GPC2",
  "gene_name": "Glypican-2"
}